{
  "term_id": "UNKNOWN:0002",
  "gene_symbol": "PYGO2",
  "gene_name": "Pygopus homolog 2",
  "term_label": "Unknown biological process",
  "gene": "UniProtKB:Q9BRQ0"
}